{
  "gene_name": "PWWP domain-containing DNA repair factor 3A",
  "term_label": "cytosol",
  "gene": "UniProtKB:Q2TAK8",
  "gene_symbol": "PWWP3A",
  "term_id": "GO:0005829"
}